{
  "term_label": "Unknown cellular component",
  "gene_symbol": "UNQ9370_PRO34162",
  "gene": "UniProtKB:Q6UXP9",
  "term_id": "UNKNOWN:0003",
  "gene_name": "Putative uncharacterized protein UNQ9370_PRO34162"
}